{
  "gene": "UniProtKB:P51878",
  "term_label": "positive regulation of inflammatory response",
  "gene_symbol": "CASP5",
  "gene_name": "Caspase-5",
  "term_id": "GO:0050729"
}